{
  "gene": "UniProtKB:Q7KZ85",
  "term_id": "GO:0034728",
  "term_label": "nucleosome organization",
  "gene_symbol": "SUPT6H",
  "gene_name": "Transcription elongation factor SPT6"
}